{
  "gene": "UniProtKB:Q8WV93",
  "term_id": "GO:0005739",
  "term_label": "mitochondrion",
  "gene_symbol": "AFG1L",
  "gene_name": "AFG1-like ATPase"
}